{
  "gene_symbol": "DEFB108C",
  "gene_name": "Putative beta-defensin 108A",
  "gene": "UniProtKB:A8MXU0",
  "term_label": "Unknown molecular function",
  "term_id": "UNKNOWN:0001"
}